{
  "gene_symbol": "MOSMO",
  "gene": "UniProtKB:Q8NHV5",
  "gene_name": "Modulator of smoothened protein",
  "term_id": "GO:0060170",
  "term_label": "ciliary membrane"
}